{
  "term_label": "cytoplasmic side of plasma membrane",
  "gene": "UniProtKB:P29074",
  "term_id": "GO:0009898",
  "gene_symbol": "PTPN4",
  "gene_name": "Tyrosine-protein phosphatase non-receptor type 4"
}